{
  "term_label": "immunoglobulin complex",
  "term_id": "GO:0019814",
  "gene_name": "Immunoglobulin kappa variable 2D-26",
  "gene": "UniProtKB:A0A0A0MRZ7",
  "gene_symbol": "IGKV2D-26"
}